{
  "term_id": "UNKNOWN:0002",
  "gene_name": "Speriolin",
  "gene_symbol": "SPATC1",
  "term_label": "Unknown biological process",
  "gene": "UniProtKB:Q76KD6"
}